{
  "term_label": "Unknown cellular component",
  "term_id": "UNKNOWN:0003",
  "gene_symbol": "RASA1",
  "gene": "UniProtKB:P20936",
  "gene_name": "Ras GTPase-activating protein 1"
}